metanephric glomerular endothelium development [GO:0072264] (biological process) Relationships: is a type of GO:0072011; is a type of GO:0072244; BFO_0000050 metanephric glomerulus vasculature development [GO:0072239] Sources: GOC:mtg_kidney_jan10 Definition: The process whose specific outcome is the progression of the metanephric glomerular endothelium over time, from its formation to the mature structure. The metanephric glomerular endothelium is an epithelial tissue that covers the internal surfaces of the glomerulus of the metanephros.